{
  "term_label": "pore-forming activity",
  "term_id": "GO:0140911",
  "gene": "UniProtKB:P59666",
  "gene_symbol": "DEFA3",
  "gene_name": "Neutrophil defensin 3"
}